{
  "term_id": "UNKNOWN:0001",
  "gene": "UniProtKB:O43866",
  "gene_name": "CD5 antigen-like",
  "term_label": "Unknown molecular function",
  "gene_symbol": "CD5L"
}